{
  "gene": "UniProtKB:O60279",
  "term_label": "Notch signaling pathway",
  "gene_name": "Sushi domain-containing protein 5",
  "gene_symbol": "SUSD5",
  "term_id": "GO:0007219"
}